(Z)-gamma-bisabolene synthase activity [GO:0052683] (molecular function) Sources: RHEA:26081 Definition: Catalysis of the reaction: 2-trans,6-trans-farnesyl diphosphate = (Z)-gamma-bisabolene + diphosphate. Also known as: (2E,6E)-farnesyl-diphosphate diphosphate-lyase [(Z)-gamma-bisabolene-forming] activity Relationships: is a type of carbon-oxygen lyase activity, acting on phosphates [GO:0016838]